{
  "term_id": "GO:0005231",
  "gene_symbol": "GLRB",
  "gene_name": "Glycine receptor subunit beta",
  "term_label": "excitatory extracellular ligand-gated monoatomic ion channel activity",
  "gene": "UniProtKB:P48167"
}